{
  "gene_name": "ADP-ribosylation factor-like protein 6",
  "gene_symbol": "ARL6",
  "term_label": "axoneme",
  "term_id": "GO:0005930",
  "gene": "UniProtKB:Q9H0F7"
}